{
  "gene_symbol": "PRSS23",
  "term_id": "UNKNOWN:0003",
  "term_label": "Unknown cellular component",
  "gene_name": "Serine protease 23",
  "gene": "UniProtKB:O95084"
}